{
  "gene_symbol": "CFAP206",
  "term_label": "regulation of cilium beat frequency",
  "gene_name": "Cilia- and flagella-associated protein 206",
  "gene": "UniProtKB:Q8IYR0",
  "term_id": "GO:0003356"
}